{
  "term_id": "UNKNOWN:0003",
  "gene_symbol": "FAM193A",
  "gene": "UniProtKB:P78312",
  "gene_name": "Protein FAM193A",
  "term_label": "Unknown cellular component"
}